{
  "term_label": "Unknown molecular function",
  "gene": "UniProtKB:Q16643",
  "term_id": "UNKNOWN:0001",
  "gene_symbol": "DBN1",
  "gene_name": "Drebrin"
}